{
  "term_id": "UNKNOWN:0002",
  "gene": "UniProtKB:P0DUD1",
  "gene_name": "Putative speedy protein E8",
  "gene_symbol": "SPDYE8",
  "term_label": "Unknown biological process"
}